{
  "term_id": "UNKNOWN:0001",
  "term_label": "Unknown molecular function",
  "gene_symbol": "Q8N7P7",
  "gene": "UniProtKB:Q8N7P7",
  "gene_name": "Uncharacterized protein FLJ40521"
}